{
  "term_label": "signaling receptor activity",
  "term_id": "GO:0038023",
  "gene_symbol": "ITGA9",
  "gene_name": "Integrin alpha-9",
  "gene": "UniProtKB:Q13797"
}